{
  "gene_name": "Proliferation marker protein Ki-67",
  "gene_symbol": "MKI67",
  "term_label": "meiotic cell cycle",
  "term_id": "GO:0051321",
  "gene": "UniProtKB:P46013"
}